{
  "gene_symbol": "HMGN4",
  "gene_name": "High mobility group nucleosome-binding domain-containing protein 4",
  "gene": "UniProtKB:O00479",
  "term_label": "nucleus",
  "term_id": "GO:0005634"
}